{
  "gene": "UniProtKB:P98170",
  "gene_name": "E3 ubiquitin-protein ligase XIAP",
  "term_label": "regulation of cell cycle",
  "term_id": "GO:0051726",
  "gene_symbol": "XIAP"
}